{
  "gene": "UniProtKB:Q7Z4F1",
  "gene_symbol": "LRP10",
  "gene_name": "Low-density lipoprotein receptor-related protein 10",
  "term_id": "UNKNOWN:0002",
  "term_label": "Unknown biological process"
}